{
  "term_id": "UNKNOWN:0003",
  "gene_name": "Uncharacterized protein C1orf87",
  "term_label": "Unknown cellular component",
  "gene_symbol": "C1orf87",
  "gene": "UniProtKB:Q8N0U7"
}